{
  "gene_name": "Solute carrier family 52, riboflavin transporter, member 2",
  "term_label": "riboflavin transmembrane transporter activity",
  "gene": "UniProtKB:Q9HAB3",
  "gene_symbol": "SLC52A2",
  "term_id": "GO:0032217"
}